{
  "gene": "UniProtKB:Q96JB8",
  "gene_symbol": "MPP4",
  "term_id": "GO:0005886",
  "term_label": "plasma membrane",
  "gene_name": "MAGUK p55 subfamily member 4"
}